{
  "term_label": "negative regulation of bone resorption",
  "term_id": "GO:0045779",
  "gene_name": "Phosphatidylinositol 3,4,5-trisphosphate 5-phosphatase 1",
  "gene_symbol": "INPP5D",
  "gene": "UniProtKB:Q92835"
}